androstenedione secretion [GO:0035941] (biological process) Sources: GOC:sl Also known as: androst-4-ene-3,17-dione secretion Definition: The regulated release of androstenedione (androst-4-ene-3,17-dione) into the circulatory system. Relationships: is a type of hormone secretion [GO:0046879]; is a type of lipid export from cell [GO:0140353] Regulation: regulated by regulation of androstenedione secretion [GO:2000837]; RO_0002212 by negative regulation of androstenedione secretion [GO:2000838]; positively regulated by positive regulation of androstenedione secretion [GO:2000839]